{
  "gene_name": "Angiopoietin-4",
  "term_label": "extracellular space",
  "term_id": "GO:0005615",
  "gene_symbol": "ANGPT4",
  "gene": "UniProtKB:Q9Y264"
}